{
  "term_label": "cytoplasm",
  "term_id": "GO:0005737",
  "gene_name": "E3 ubiquitin-protein ligase XIAP",
  "gene": "UniProtKB:P98170",
  "gene_symbol": "XIAP"
}